{
  "gene": "UniProtKB:Q92523",
  "gene_name": "Carnitine O-palmitoyltransferase 1, muscle isoform",
  "gene_symbol": "CPT1B",
  "term_id": "GO:0006631",
  "term_label": "fatty acid metabolic process"
}